{
  "term_id": "GO:0006511",
  "term_label": "ubiquitin-dependent protein catabolic process",
  "gene_name": "Protein ARK2N",
  "gene_symbol": "ARK2N",
  "gene": "UniProtKB:Q96B23"
}